{
  "term_id": "UNKNOWN:0003",
  "gene_symbol": "PRR27",
  "gene": "UniProtKB:Q6MZM9",
  "gene_name": "Proline-rich protein 27",
  "term_label": "Unknown cellular component"
}